long-chain fatty acid import into cell [GO:0044539] (biological process) Relationships: is a type of long-chain fatty acid transport [GO:0015909]; is a type of import into cell [GO:0098657]; is a type of lipid import into cell [GO:0140354] Regulation: regulated by regulation of long-chain fatty acid import into cell [GO:0140212]; negatively regulated by negative regulation of long-chain fatty acid import into cell [GO:0140213]; positively regulated by positive regulation of long-chain fatty acid import into cell [GO:0140214] Also known as: long-chain fatty acid uptake, long-chain fatty acid import Note: While there is not universal consensus on the lengths of short-, medium-, long- and very-long-chain fatty acids, the GO uses the definitions in ChEBI (see CHEBI:26666, CHEBI:59554, CHEBI:15904 and CHEBI:27283). Definition: The directed movement of a long-chain fatty acid from outside of a cell into a cell. This may occur via transport across the plasma membrane or via endocytosis. A long-chain fatty acid has an aliphatic tail containing 13 to 22 carbons. Subtypes: long-chain fatty acid import across plasma membrane [GO:0015911] References: PMID:22022213 Sources: GOC:jl, GOC:pm